{
  "gene_symbol": "SPOP",
  "gene": "UniProtKB:O43791",
  "term_id": "GO:0031625",
  "term_label": "ubiquitin protein ligase binding",
  "gene_name": "Speckle-type POZ protein"
}